mesenchymal-epithelial cell signaling involved in lung development [GO:0060496] (biological process) Definition: Any process that mediates the transfer of information from a mesenchymal cell to an epithelial cell and contributes to the development of the lung. Sources: GOC:dph, GOC:mtg_lung Also known as: mesenchymal-epithelial cell signalling involved in lung development Relationships: is a type of cell-cell signaling involved in lung development [GO:0060495]; is a type of mesenchymal-epithelial cell signaling [GO:0060638] Subtypes: mesenchymal-endodermal cell signaling involved in lung induction [GO:0060493]